{
  "term_label": "plasma membrane",
  "term_id": "GO:0005886",
  "gene": "UniProtKB:Q6F5E8",
  "gene_name": "Capping protein, Arp2_3 and myosin-I linker protein 2",
  "gene_symbol": "CARMIL2"
}